{
  "gene": "UniProtKB:Q4V328",
  "gene_symbol": "GRIPAP1",
  "term_label": "Unknown molecular function",
  "gene_name": "GRIP1-associated protein 1",
  "term_id": "UNKNOWN:0001"
}